{
  "term_label": "phagophore assembly site",
  "gene_name": "Serine_threonine-protein kinase ULK2",
  "gene": "UniProtKB:Q8IYT8",
  "term_id": "GO:0000407",
  "gene_symbol": "ULK2"
}